{
  "term_label": "peroxisome organization",
  "gene_name": "Lysosomal cobalamin transporter ABCD4",
  "gene": "UniProtKB:O14678",
  "gene_symbol": "ABCD4",
  "term_id": "GO:0007031"
}